{
  "gene_symbol": "MAPK1",
  "gene_name": "Mitogen-activated protein kinase 1",
  "term_id": "GO:0035556",
  "gene": "UniProtKB:P28482",
  "term_label": "intracellular signal transduction"
}